nuclear histone mRNA catabolic process [GO:0071045] (biological process) Definition: The chemical reactions and pathways resulting in the breakdown of histone messenger RNA (mRNA) within the nucleus. References: PMID:17179095, PMID:17855393 Sources: GOC:dgf, GOC:krc Relationships: is a type of GO:0071044